{
  "term_id": "UNKNOWN:0003",
  "gene_symbol": "ZMYM2",
  "gene": "UniProtKB:Q9UBW7",
  "gene_name": "Zinc finger MYM-type protein 2",
  "term_label": "Unknown cellular component"
}